{
  "term_id": "GO:0061459",
  "gene_name": "Cationic amino acid transporter 2",
  "gene_symbol": "SLC7A2",
  "gene": "UniProtKB:P52569",
  "term_label": "L-arginine transmembrane transporter activity"
}